thiol oxidase activity [GO:0016972] (molecular function) Relationships: is a type of GO:0015036; is a type of oxidoreductase activity, acting on a sulfur group of donors, oxygen as acceptor [GO:0016670] Sources: RHEA:17357 Subtypes: flavin-dependent sulfhydryl oxidase activity [GO:0016971] Definition: Catalysis of the reaction: 2 R'C(R)SH + O2 = R'C(R)S-S(R)CR' + 2 H2O2. Also known as: sulfhydryl oxidase activity, thiol:oxygen oxidoreductase activity